{
  "term_id": "GO:0033781",
  "gene_symbol": "CYP46A1",
  "term_label": "cholesterol 24-hydroxylase activity",
  "gene": "UniProtKB:Q9Y6A2",
  "gene_name": "Cholesterol 24-hydroxylase"
}